{
  "term_label": "secretory vesicle",
  "gene": "UniProtKB:P61026",
  "gene_symbol": "RAB10",
  "gene_name": "Ras-related protein Rab-10",
  "term_id": "GO:0099503"
}